negative regulation of plasma kallikrein-kinin cascade [GO:0002549] (biological process) Definition: Any process that stops, prevents, or reduces the frequency, rate, or extent of the plasma kallikrein-kinin cascade. Relationships: is a type of negative regulation of kinin cascade [GO:0002257]; is a type of regulation of plasma kallikrein-kinin cascade [GO:0002529]; negatively regulates plasma kallikrein-kinin cascade [GO:0002353] Sources: GOC:add Also known as: down regulation of plasma kallikrein-kinin cascade, down-regulation of plasma kallikrein-kinin cascade, downregulation of plasma kallikrein-kinin cascade, inhibition of plasma kallikrein-kinin cascade